negative regulation of intrinsic apoptotic signaling pathway in response to osmotic stress [GO:1902219] (biological process) Also known as: down regulation of intrinsic apoptotic signaling pathway in response to osmotic stress, down-regulation of intrinsic apoptotic signaling pathway in response to osmotic stress, downregulation of intrinsic apoptotic signaling pathway in response to osmotic stress, inhibition of intrinsic apoptotic signaling pathway in response to osmotic stress Subtypes: negative regulation of intrinsic apoptotic signaling pathway in response to osmotic stress by p53 class mediator [GO:1902239] Relationships: is a type of regulation of intrinsic apoptotic signaling pathway in response to osmotic stress [GO:1902218]; is a type of negative regulation of intrinsic apoptotic signaling pathway [GO:2001243]; negatively regulates intrinsic apoptotic signaling pathway in response to osmotic stress [GO:0008627] References: PMID:14569084 Sources: GOC:BHF, GOC:TermGenie, GOC:mtg_apoptosis, GOC:rl Definition: Any process that stops, prevents or reduces the frequency, rate or extent of intrinsic apoptotic signaling pathway in response to osmotic stress.